{
  "term_label": "actomyosin structure organization",
  "term_id": "GO:0031032",
  "gene": "UniProtKB:A2A2Y4",
  "gene_symbol": "FRMD3",
  "gene_name": "FERM domain-containing protein 3"
}